{
  "term_id": "GO:0005267",
  "gene_symbol": "ABCC9",
  "gene_name": "ATP-binding cassette sub-family C member 9",
  "term_label": "potassium channel activity",
  "gene": "UniProtKB:O60706"
}